t-circle formation [GO:0090656] (BP) Definition: A telomere maintenance process that results in the formation of a telomeric circle, or t-circle. A t-circle is an extrachromosomal duplex or single-stranded circular DNA molecule composed of t-arrays. T-circles are involved in the control of telomere length via alternative-lengthening of telomeres (ALT) pathway and telomere rapid deletion (TRD). Relationships: is a type of formation of extrachromosomal circular DNA [GO:0001325]; is part of GO:0090737 References: PMID:19214183, PMID:19581589, PMID:19809492, PMID:19858100 Sources: GOC:BHF, GOC:BHF_telomere, GOC:nc Regulation: regulated by GO:1904429; negatively regulated by negative regulation of t-circle formation [GO:1904430]; positively regulated by GO:1904431 Also known as: telomeric circle formation